lymphocyte aggregation [GO:0071593] (biological process) Definition: The adhesion of one lymphocyte to one or more other lymphocytes via adhesion molecules. Subtypes: T cell aggregation [GO:0070489] Relationships: is a type of leukocyte aggregation [GO:0070486] Sources: GOC:sl